{
  "gene_symbol": "RHOT2",
  "term_id": "GO:0005741",
  "gene_name": "Mitochondrial Rho GTPase 2",
  "gene": "UniProtKB:Q8IXI1",
  "term_label": "mitochondrial outer membrane"
}